response to oscillatory fluid shear stress [GO:0097702] (biological process) Subtypes: cellular response to oscillatory fluid shear stress [GO:0097704] Definition: Any response to fluid shear stress where the fluid is moving across a solid surface with an oscillatory flow. Disturbed flow patterns at the arterial bifurcations and curvatures may cause endothelial dysfunction, which initiates atherosclerosis. References: PMID:21768538 Sources: GOC:BHF, GOC:BHF_miRNA, GOC:bc Relationships: is_a GO:0034405